{
  "gene": "UniProtKB:Q9UG01",
  "gene_symbol": "IFT172",
  "term_id": "GO:0005930",
  "term_label": "axoneme",
  "gene_name": "Intraflagellar transport protein 172 homolog"
}